intermediate mesoderm morphogenesis [GO:0048390] (biological process) Sources: GOC:go_curators Relationships: is a type of mesoderm morphogenesis [GO:0048332]; is part of GO:0048389 Definition: The process in which the anatomical structures of the intermediate mesoderm are generated and organized.